{
  "term_id": "GO:0021987",
  "term_label": "cerebral cortex development",
  "gene_name": "Transforming acidic coiled-coil-containing protein 1",
  "gene_symbol": "TACC1",
  "gene": "UniProtKB:O75410"
}